{
  "gene_symbol": "PAGR1",
  "term_label": "positive regulation of cell cycle G1/S phase transition",
  "gene": "UniProtKB:Q9BTK6",
  "term_id": "GO:1902808",
  "gene_name": "PAXIP1-associated glutamate-rich protein 1"
}